{
  "gene_symbol": "AGO3",
  "term_label": "regulatory ncRNA-mediated post-transcriptional gene silencing",
  "term_id": "GO:0035194",
  "gene_name": "Protein argonaute-3",
  "gene": "UniProtKB:Q9H9G7"
}